{
  "term_label": "RNA polymerase II general transcription initiation factor activity",
  "term_id": "GO:0016251",
  "gene_symbol": "TAF4B",
  "gene_name": "Transcription initiation factor TFIID subunit 4B",
  "gene": "UniProtKB:Q92750"
}